{
  "term_id": "GO:0060369",
  "gene_name": "CD226 antigen",
  "gene": "UniProtKB:Q15762",
  "gene_symbol": "CD226",
  "term_label": "positive regulation of Fc receptor mediated stimulatory signaling pathway"
}